{
  "gene_symbol": "AGBL4",
  "term_label": "cytoplasm",
  "gene": "UniProtKB:Q5VU57",
  "gene_name": "Cytosolic carboxypeptidase 6",
  "term_id": "GO:0005737"
}